N-acetyllactosamine beta-1,3-glucuronosyltransferase activity [GO:0046987] (molecular function) Definition: Catalysis of the transfer, in a beta 1,3 linkage, of D-glucuronic acid (GlcUA) from UDP-D-glucuronic acid to N-acetyllactosamine (galactosyl beta-1,4-N-acetylglucosamine). References: PMID:12511570 Sources: GOC:bf Relationships: is_a glucuronosyltransferase activity [GO:0015020] Also known as: galactosyl beta-1,4 N-acetylglucosamine beta-1,3 glucuronosyltransferase activity